negative regulation of cell activation [GO:0050866] (biological process) Definition: Any process that stops, prevents, or reduces the frequency, rate or extent of cell activation. Also known as: down regulation of cell activation, down-regulation of cell activation, downregulation of cell activation, inhibition of cell activation Sources: GOC:ai Subtypes: negative regulation of leukocyte activation [GO:0002695], negative regulation of platelet activation [GO:0010544], GO:0061889, negative regulation of skeletal muscle satellite cell activation involved in skeletal muscle regeneration [GO:1901667], GO:1904988, negative regulation of hepatic stellate cell activation [GO:2000490] Relationships: is a type of GO:0048523; is a type of regulation of cell activation [GO:0050865]; is a type of negative regulation of multicellular organismal process [GO:0051241]; negatively regulates cell activation [GO:0001775]